{
  "gene": "UniProtKB:Q13507",
  "term_label": "inositol 1,4,5 trisphosphate binding",
  "gene_name": "Short transient receptor potential channel 3",
  "term_id": "GO:0070679",
  "gene_symbol": "TRPC3"
}